{
  "term_id": "UNKNOWN:0002",
  "gene_symbol": "IGF2BP2-AS1",
  "term_label": "Unknown biological process",
  "gene_name": "Putative uncharacterized protein IGF2BP2-AS1",
  "gene": "UniProtKB:Q96M15"
}